{
  "gene_name": "Tyrosine-protein kinase Mer",
  "gene_symbol": "MERTK",
  "term_label": "nervous system development",
  "gene": "UniProtKB:Q12866",
  "term_id": "GO:0007399"
}